{
  "gene_name": "Rhomboid-related protein 2",
  "term_label": "Unknown biological process",
  "gene_symbol": "RHBDL2",
  "gene": "UniProtKB:Q9NX52",
  "term_id": "UNKNOWN:0002"
}